{
  "gene": "UniProtKB:P05019",
  "term_id": "GO:0005179",
  "gene_symbol": "IGF1",
  "gene_name": "Insulin-like growth factor I",
  "term_label": "hormone activity"
}